positive regulation of circadian sleep/wake cycle, REM sleep [GO:0046005] (biological process) Also known as: positive regulation of REM sleep, up regulation of circadian sleep/wake cycle, REM sleep, up-regulation of circadian sleep/wake cycle, REM sleep, upregulation of circadian sleep/wake cycle, REM sleep, activation of circadian sleep/wake cycle, REM sleep, stimulation of circadian sleep/wake cycle, REM sleep Sources: GOC:go_curators Definition: Any process that activates or increases the duration or quality of rapid eye movement (REM) sleep. Relationships: is a type of GO:0042320; is a type of positive regulation of circadian sleep/wake cycle, sleep [GO:0045938]; positively regulates GO:0042747